{
  "gene_symbol": "CACNB4",
  "term_id": "GO:0005891",
  "term_label": "voltage-gated calcium channel complex",
  "gene": "UniProtKB:O00305",
  "gene_name": "Voltage-dependent L-type calcium channel subunit beta-4"
}